cellular response to interleukin-8 [GO:0098759] (biological process) Definition: Any process that results in a change in state or activity of a cell (in terms of movement, secretion, enzyme production, gene expression, etc.) as a result of an interleukin-8 stimulus. Also known as: cellular response to IL-8 Sources: GOC:BHF, GOC:mah Relationships: is a type of GO:0071345; is a type of response to interleukin-8 [GO:0098758]